{
  "gene_name": "18S rRNA aminocarboxypropyltransferase",
  "gene_symbol": "TSR3",
  "gene": "UniProtKB:Q9UJK0",
  "term_id": "GO:0030490",
  "term_label": "maturation of SSU-rRNA"
}